opioid receptor binding [GO:0031628] (molecular function) Definition: Binding to an opioid receptor. Sources: GOC:nln Relationships: is a type of G protein-coupled receptor binding [GO:0001664] Subtypes: delta-type opioid receptor binding [GO:0031850], GO:0031851, mu-type opioid receptor binding [GO:0031852], nociceptin receptor binding [GO:0031853]